{
  "term_label": "protein serine/threonine kinase activity",
  "term_id": "GO:0004674",
  "gene_symbol": "MOK",
  "gene_name": "MAPK_MAK_MRK overlapping kinase",
  "gene": "UniProtKB:Q9UQ07"
}